{
  "term_id": "UNKNOWN:0002",
  "gene_name": "Olfactory receptor 52L1",
  "term_label": "Unknown biological process",
  "gene_symbol": "OR52L1",
  "gene": "UniProtKB:Q8NGH7"
}